host cell centrosome [GO:0120148] (cellular component) Also known as: host centrosome Definition: A structure in a host cell comprised of a core structure (in most organisms, a pair of centrioles) and peripheral material from which a microtubule-based structure, such as a spindle apparatus, is organized. Centrosomes occur close to the nucleus during interphase in many eukaryotic cells, though in animal cells it changes continually during the cell-division cycle. Sources: ISBN:0198547684 Relationships: is a type of host cytoskeleton [GO:0044163]